{
  "term_label": "protein kinase activity",
  "gene_name": "Mitogen-activated protein kinase kinase kinase 21",
  "term_id": "GO:0004672",
  "gene": "UniProtKB:Q5TCX8",
  "gene_symbol": "MAP3K21"
}